negative regulation of cellular response to manganese ion [GO:1905803] (biological process) Definition: Any process that stops, prevents or reduces the frequency, rate or extent of cellular response to manganese ion. References: PMID:23721876 Sources: GOC:TermGenie, GO_REF:0000058 Also known as: down regulation of cellular response to manganese, down regulation of cellular response to manganese ion, down-regulation of cellular response to manganese, down-regulation of cellular response to manganese ion, downregulation of cellular response to manganese, downregulation of cellular response to manganese ion, negative regulation of cellular response to manganese, inhibition of cellular response to manganese, inhibition of cellular response to manganese ion Relationships: is a type of GO:0048523; is a type of negative regulation of response to stimulus [GO:0048585]; is a type of GO:1905802; negatively regulates cellular response to manganese ion [GO:0071287]